{
  "gene": "UniProtKB:Q9H7X0",
  "term_id": "GO:0007059",
  "term_label": "chromosome segregation",
  "gene_name": "N-alpha-acetyltransferase 60",
  "gene_symbol": "NAA60"
}